pantothenate kinase activity [GO:0004594] (MF) Sources: EC:2.7.1.33 Relationships: is a type of kinase activity [GO:0016301]; is a type of GO:0016773 Also known as: ATP:(R)-pantothenate 4'-phosphotransferase activity, ATP:pantothenate 4'-phosphotransferase activity, D-pantothenate kinase activity, pantothenate kinase (phosphorylating) activity, pantothenic acid kinase activity Definition: Catalysis of the reaction: ATP + pantothenate = ADP + D-4'-phosphopantothenate.